granuloma formation [GO:0002432] (biological process) Relationships: is a type of immune effector process [GO:0002252]; BFO_0000050 GO:0002544 Regulation: regulated by regulation of granuloma formation [GO:0002631]; negatively regulated by negative regulation of granuloma formation [GO:0002632]; positively regulated by positive regulation of granuloma formation [GO:0002633] Sources: GOC:add, GO_REF:0000022, ISBN:068340007X, ISBN:0721601464, ISBN:081533642X Definition: The formation of nodular inflammatory lesions, usually small or granular, firm, persistent, well-structured, and containing compactly grouped T lymphocytes and modified phagocytes such as epithelioid cells, giant cells, and other macrophages. Granuloma formation represents a chronic inflammatory response initiated by various infectious and noninfectious agents. The center of a granuloma consists of fused macrophages, which can become necrotic.